{
  "term_id": "GO:0000139",
  "gene_symbol": "NAA60",
  "term_label": "Golgi membrane",
  "gene_name": "N-alpha-acetyltransferase 60",
  "gene": "UniProtKB:Q9H7X0"
}